{
  "gene_symbol": "ZNF287",
  "term_id": "GO:0000978",
  "gene_name": "Zinc finger protein 287",
  "gene": "UniProtKB:Q9HBT7",
  "term_label": "RNA polymerase II cis-regulatory region sequence-specific DNA binding"
}